{
  "gene_name": "Serine_arginine-rich splicing factor 6",
  "term_label": "mRNA binding",
  "gene": "UniProtKB:Q13247",
  "gene_symbol": "SRSF6",
  "term_id": "GO:0003729"
}